mitotic telophase [GO:0000093] (biological process) Sources: GOC:mtg_cell_cycle Note: Note that this term should not be used for direct annotation. If you are trying to make an annotation to x phase, it is likely that the correct annotation is 'regulation of x/y phase transition' or to a process which occurs during the reported phase (i.e mitotic DNA replication for mitotic S-phase). To capture the phase when a specific location or process is observed, the phase term can be used in an annotation extension (PMID:24885854) applied to a cellular component term (with the relation exists_during) or a biological process term (with the relation happens_during). Definition: The cell cycle phase which follows anaphase during M phase of mitosis and during which the chromosomes arrive at the poles of the cell and the division of the cytoplasm starts. Relationships: is a type of telophase [GO:0051326]; is part of mitotic M phase [GO:0000087]